16S rRNA pseudouridine(516) synthase activity [GO:0160136] (MF) Relationships: is a type of rRNA pseudouridine synthase activity [GO:0120159] Sources: EC:5.4.99.19, RHEA:38867 Definition: Catalysis of the reaction: uridine(516) in 16S rRNA = pseudouridine(516) in 16S rRNA.